{
  "term_label": "signaling receptor activity",
  "gene_name": "Reticulon-4 receptor-like 1",
  "term_id": "GO:0038023",
  "gene": "UniProtKB:Q86UN2",
  "gene_symbol": "RTN4RL1"
}